{
  "term_label": "sequestering of BMP in extracellular matrix",
  "gene_symbol": "DAND5",
  "term_id": "GO:0035582",
  "gene": "UniProtKB:Q8N907",
  "gene_name": "DAN domain family member 5"
}